positive regulation of protein linear polyubiquitination [GO:1902530] (biological process) Definition: Any process that activates or increases the frequency, rate or extent of protein linear polyubiquitination. Note: An example is BIRC2 (UniProt ID Q13490) in PMID:21931591. References: PMID:21931591 Sources: GOC:TermGenie Relationships: is_a regulation of protein linear polyubiquitination [GO:1902528]; is a type of positive regulation of protein polyubiquitination [GO:1902916]; positively regulates GO:0097039 Also known as: up regulation of protein linear polyubiquitination, up-regulation of protein linear polyubiquitination, upregulation of protein linear polyubiquitination, activation of M1 linkage, activation of protein linear polyubiquitination, positive regulation of M1 linkage, up regulation of M1 linkage, up-regulation of M1 linkage, upregulation of M1 linkage